{
  "term_id": "GO:0005886",
  "gene_symbol": "HRH1",
  "term_label": "plasma membrane",
  "gene_name": "Histamine H1 receptor",
  "gene": "UniProtKB:P35367"
}